negative regulation of chemokine (C-C motif) ligand 1 production [GO:0071653] (biological process) Definition: Any process that stops, prevents, or reduces the frequency, rate, or extent of production of chemokine (C-C motif) ligand 1. Sources: GOC:mah Relationships: is a type of GO:0032682; is a type of GO:0071652; negatively regulates GO:0071610 Also known as: negative regulation of CCL1 production, negative regulation of T cell activation 3 production, negative regulation of TCA-3 production